{
  "gene_name": "Interleukin-1 receptor-associated kinase 3",
  "gene_symbol": "IRAK3",
  "gene": "UniProtKB:Q9Y616",
  "term_id": "GO:0005737",
  "term_label": "cytoplasm"
}